embryo sac nuclear migration [GO:0009562] (biological process) Subtypes: nuclear migration to embryo sac poles [GO:0023002], nuclear migration to the embryo sac center [GO:0023003] Relationships: is a type of GO:0007097; is part of megagametogenesis [GO:0009561] Sources: GOC:jl, GOC:mtg_plant Definition: The directed movement of an embryo sac nucleus to the pole or center of the cell. Also known as: embryo sac nucleus migration, female gametophyte nuclear migration, female gametophyte nucleus migration, megagametophyte nuclear migration, megagametophyte nucleus migration